{
  "term_id": "GO:0044281",
  "term_label": "small molecule metabolic process",
  "gene_symbol": "L2HGDH",
  "gene": "UniProtKB:Q9H9P8",
  "gene_name": "L-2-hydroxyglutarate dehydrogenase, mitochondrial"
}